{
  "gene_symbol": "PRAMEF11",
  "gene_name": "PRAME family member 11",
  "term_label": "Cul2-RING ubiquitin ligase complex",
  "term_id": "GO:0031462",
  "gene": "UniProtKB:O60813"
}